{
  "term_label": "transcription initiation at RNA polymerase II promoter",
  "gene": "UniProtKB:P36954",
  "term_id": "GO:0006367",
  "gene_symbol": "POLR2I",
  "gene_name": "DNA-directed RNA polymerase II subunit RPB9"
}